granulocyte colony-stimulating factor receptor activity [GO:0004902] (molecular function) Sources: GOC:mah, GOC:signaling Also known as: G-CSF receptor activity, granulocyte colony stimulating factor receptor activity, CSF3R Definition: Combining with granulocyte colony-stimulating factor (G-CSF) and transmitting the signal from one side of the membrane to the other to initiate a change in cell activity. Relationships: is a type of cytokine receptor activity [GO:0004896]; is part of GO:0038158; has part GO:0051916